{
  "term_id": "GO:0006357",
  "term_label": "regulation of transcription by RNA polymerase II",
  "gene_name": "Mitotic deacetylase-associated SANT domain protein",
  "gene_symbol": "MIDEAS",
  "gene": "UniProtKB:Q6PJG2"
}